maintenance of RNA location [GO:0051237] (biological process) Subtypes: GO:0046594 Relationships: is a type of maintenance of location [GO:0051235]; is part of GO:0006403 Also known as: RNA retention, maintenance of RNA localization Definition: Any process in which RNA is maintained in a location and prevented from moving elsewhere. Sources: GOC:ai